{
  "term_id": "GO:0000981",
  "gene_name": "Zinc finger and BTB domain-containing protein 22",
  "gene_symbol": "ZBTB22",
  "gene": "UniProtKB:O15209",
  "term_label": "DNA-binding transcription factor activity, RNA polymerase II-specific"
}